{
  "term_id": "GO:0031175",
  "gene": "UniProtKB:Q13740",
  "term_label": "neuron projection development",
  "gene_name": "CD166 antigen",
  "gene_symbol": "ALCAM"
}